{
  "term_label": "clathrin complex",
  "gene": "UniProtKB:Q00610",
  "gene_symbol": "CLTC",
  "term_id": "GO:0071439",
  "gene_name": "Clathrin heavy chain 1"
}